Nkx-2.5 complex [GO:1990664] (cellular component) Note: An example of this is Nkx-2.5 in human (UniProt symbol P52952) in PMID:22849347 (inferred from direct assay). References: PMID:22849347 Sources: GOC:ame Relationships: is a type of RNA polymerase II transcription regulator complex [GO:0090575] Definition: A transcription factor complex formed by two or more subunits of Nkx-2.5. Nkx-2.5 is an evolutionary conserved transcription factor important for the specification and differentiation of cardiomyocytes during heart development. It is also required for spleen development. It binds DNA either as a monomer, or a homodimer, or a heterodimer complex to activate or inhibit expression of genes. Also known as: Nkx-2.5 homodimer complex, NKX.2-5 homodimer complex, NKX2.5 complex, NKX2E homodimer complex